{
  "term_id": "GO:0007166",
  "gene": "UniProtKB:P11836",
  "gene_name": "B-lymphocyte antigen CD20",
  "gene_symbol": "MS4A1",
  "term_label": "cell surface receptor signaling pathway"
}